{
  "gene": "UniProtKB:Q13398",
  "gene_name": "Zinc finger protein 211",
  "term_label": "DNA-binding transcription factor activity, RNA polymerase II-specific",
  "gene_symbol": "ZNF211",
  "term_id": "GO:0000981"
}